regulation of anaphase-promoting complex-dependent catabolic process [GO:1905784] (biological process) References: PMID:10921876 Sources: GOC:TermGenie, GO_REF:0000058 Relationships: is a type of regulation of proteasomal ubiquitin-dependent protein catabolic process [GO:0032434]; regulates anaphase-promoting complex-dependent catabolic process [GO:0031145] Subtypes: negative regulation of anaphase-promoting complex-dependent catabolic process [GO:1905785], GO:1905786 Definition: Any process that modulates the frequency, rate or extent of anaphase-promoting complex-dependent catabolic process.